{
  "gene_symbol": "KNDC1",
  "term_id": "GO:0005085",
  "term_label": "guanyl-nucleotide exchange factor activity",
  "gene": "UniProtKB:Q76NI1",
  "gene_name": "Kinase non-catalytic C-lobe domain-containing protein 1"
}